altronate dehydratase activity [GO:0008789] (molecular function) Sources: EC:4.2.1.7, RHEA:15957 Also known as: D-altronate hydro-lyase (2-dehydro-3-deoxy-D-galactonate-forming), D-altronate hydro-lyase activity Definition: Catalysis of the reaction: D-altronate = 2-dehydro-3-deoxy-D-gluconate + H2O. Relationships: is a type of hydro-lyase activity [GO:0016836]